2-halobenzoate 1,2-dioxygenase activity [GO:0018626] (molecular function) Also known as: 2-chlorobenzoate 1,2-dioxygenase activity, 2-chlorobenzoate,NADH:oxygen oxidoreductase (1,2-hydroxylating, dechlorinating, decarboxylating) Definition: Catalysis of the reaction: a 2-halobenzoate + NADH + O2 + H+ = a halide anion + catechol + CO2 + NAD+. Sources: RHEA:53736 Relationships: is a type of oxidoreductase activity, acting on paired donors, with incorporation or reduction of molecular oxygen, NAD(P)H as one donor, and incorporation of two atoms of oxygen into one donor [GO:0016708]